{
  "term_label": "cytosol",
  "term_id": "GO:0005829",
  "gene": "UniProtKB:Q9BVM4",
  "gene_name": "Gamma-glutamylaminecyclotransferase",
  "gene_symbol": "GGACT"
}